{
  "term_label": "plasma membrane",
  "gene": "UniProtKB:Q9Y2T6",
  "term_id": "GO:0005886",
  "gene_name": "G-protein coupled receptor 55",
  "gene_symbol": "GPR55"
}